{
  "term_label": "3'-UTR-mediated mRNA destabilization",
  "gene_name": "Probable ribonuclease ZC3H12B",
  "gene_symbol": "ZC3H12B",
  "term_id": "GO:0061158",
  "gene": "UniProtKB:Q5HYM0"
}